{
  "term_label": "liver development",
  "term_id": "GO:0001889",
  "gene": "UniProtKB:Q9HAW7",
  "gene_name": "UDP-glucuronosyltransferase 1A7",
  "gene_symbol": "UGT1A7"
}